{
  "gene": "UniProtKB:P22413",
  "gene_name": "Ectonucleotide pyrophosphatase_phosphodiesterase family member 1",
  "gene_symbol": "ENPP1",
  "term_id": "GO:0030505",
  "term_label": "inorganic diphosphate transport"
}